{
  "gene_symbol": "NPEPPS",
  "term_id": "GO:0005576",
  "gene": "UniProtKB:P55786",
  "term_label": "extracellular region",
  "gene_name": "Puromycin-sensitive aminopeptidase"
}